response to triacyl bacterial lipopeptide [GO:0071725] (BP) Definition: Any process that results in a change in state or activity of a cell or an organism (in terms of movement, secretion, enzyme production, gene expression, etc.) as a result of a triacylated bacterial lipopeptide stimulus. References: PMID:12077222, PMID:12524386, PMID:2757794 Sources: GOC:add Relationships: is a type of response to bacterial lipopeptide [GO:0070339] Note: Note that bacterial lipopeptides are derived from bacterial lipoproteins, but the two terms are sometimes used interchangeably in the literature. Also known as: response to triacylated bacterial lipoprotein Subtypes: detection of triacyl bacterial lipopeptide [GO:0042495], cellular response to triacyl bacterial lipopeptide [GO:0071727]